positive regulation of non-canonical NF-kappaB signal transduction [GO:1901224] (biological process) Also known as: up-regulation of noncanonical NF-kappaB signaling, upregulation of noncanonical NF-kappaB signaling, activation of non-canonical NF-KB signaling, activation of noncanonical NF-kappaB signaling, activation of noncanonical nuclear factor kappaB (NF-kappaB) pathway, positive regulation of NIK/NF-kappaB cascade, positive regulation of NIK/NF-kappaB signaling, positive regulation of non-canonical NF-KB signaling, positive regulation of noncanonical NF-kappaB signaling, positive regulation of noncanonical nuclear factor kappaB (NF-kappaB) pathway, up regulation of NIK/NF-kappaB cascade, up regulation of non-canonical NF-KB signaling, up regulation of noncanonical NF-kappaB signaling, up regulation of noncanonical nuclear factor kappaB (NF-kappaB) pathway, up-regulation of non-canonical NF-KB signaling, up-regulation of noncanonical nuclear factor kappaB (NF-kappaB) pathway, upregulation of NIK/NF-kappaB cascade, upregulation of non-canonical NF-KB signaling, upregulation of noncanonical nuclear factor kappaB (NF-kappaB) pathway, activation of NIK/NF-kappaB cascade, activation of p52-dependent NF-kappaB signaling, positive regulation of NF-kappaB import into nucleus, positive regulation of p52-dependent NF-kappaB signaling, up regulation of p52-dependent NF-kappaB signaling, up-regulation of p52-dependent NF-kappaB signaling, upregulation of p52-dependent NF-kappaB signaling, up-regulation of NIK/NF-kappaB cascade Definition: Any process that activates or increases the frequency, rate or extent of the non-canonical NF-kappaB cascade. Sources: GOC:TermGenie Relationships: is_a regulation of non-canonical NF-kappaB signal transduction [GO:1901222]; is_a GO:1902533; positively regulates non-canonical NF-kappaB signal transduction [GO:0038061]